{
  "term_id": "GO:0000978",
  "term_label": "RNA polymerase II cis-regulatory region sequence-specific DNA binding",
  "gene_symbol": "JDP2",
  "gene_name": "Jun dimerization protein 2",
  "gene": "UniProtKB:Q8WYK2"
}